{
  "gene_name": "Large ribosomal subunit protein uL29m",
  "gene_symbol": "MRPL47",
  "gene": "UniProtKB:Q9HD33",
  "term_label": "structural constituent of ribosome",
  "term_id": "GO:0003735"
}